{
  "gene_name": "Cyclin-dependent kinase 12",
  "gene": "UniProtKB:Q9NYV4",
  "term_label": "cyclin/CDK positive transcription elongation factor complex",
  "term_id": "GO:0008024",
  "gene_symbol": "CDK12"
}